{
  "term_id": "GO:0099645",
  "gene": "UniProtKB:Q8TDF5",
  "gene_name": "Neuropilin and tolloid-like protein 1",
  "term_label": "neurotransmitter receptor localization to postsynaptic specialization membrane",
  "gene_symbol": "NETO1"
}